instar larval or pupal development [GO:0002165] (biological process) Sources: GOC:jid, GOC:mtg_sensu Definition: The process whose specific outcome is the progression of the instar larva or pupa over time, from its formation to the mature structure. An example of this process is found in Drosophila melanogaster. Subtypes: GO:0002168, pupal development [GO:0035209], GO:0035210 Relationships: is a type of multicellular organism development [GO:0007275]; is_a post-embryonic development [GO:0009791]